{
  "gene": "UniProtKB:Q9UNK9",
  "term_label": "Unknown biological process",
  "gene_symbol": "ANGEL1",
  "gene_name": "Protein angel homolog 1",
  "term_id": "UNKNOWN:0002"
}